{
  "term_label": "nucleoplasm",
  "gene": "UniProtKB:O14497",
  "term_id": "GO:0005654",
  "gene_symbol": "ARID1A",
  "gene_name": "AT-rich interactive domain-containing protein 1A"
}